(1->4)-beta-D-galactan binding [GO:2001081] (molecular function) Sources: GOC:mengo_curators Relationships: is a type of polysaccharide binding [GO:0030247] Definition: Binding to (1->4)-beta-D-galactan. Also known as: (1,4)-beta-D-galactan binding